detection of carbon dioxide by vasomotor center [GO:0002013] (biological process) Definition: The process by a carbon dioxide stimulus is received and converted to a molecular signal by the vasomotor center of the central nervous system. Relationships: is a type of detection of carbon dioxide [GO:0003031]; is part of GO:0001980 Sources: ISBN:0721643949